{
  "term_id": "GO:0051294",
  "gene": "UniProtKB:Q6P1M3",
  "gene_name": "LLGL scribble cell polarity complex component 2",
  "term_label": "establishment of spindle orientation",
  "gene_symbol": "LLGL2"
}